{
  "gene_symbol": "Q6ZVU0",
  "gene": "UniProtKB:Q6ZVU0",
  "term_label": "Unknown cellular component",
  "term_id": "UNKNOWN:0003",
  "gene_name": "Putative uncharacterized protein FLJ42102"
}